monoatomic cation homeostasis [GO:0055080] (biological process) Also known as: cation homeostasis Definition: Any process involved in the maintenance of an internal steady state of monoatomic cations within an organism or cell. Monatomic cations (also called simple cations) are cations consisting of exactly one atom. Relationships: is a type of monoatomic ion homeostasis [GO:0050801] Sources: GOC:ceb, GOC:jid, GOC:mah Subtypes: regulation of pH [GO:0006885], GO:0010960, intracellular monoatomic cation homeostasis [GO:0030003], copper ion homeostasis [GO:0055070], GO:0055071, calcium ion homeostasis [GO:0055074], GO:0055075, sodium ion homeostasis [GO:0055078], GO:0060586